{
  "gene_name": "TP53-target gene 3 protein",
  "gene_symbol": "TP53TG3F",
  "term_id": "UNKNOWN:0002",
  "term_label": "Unknown biological process",
  "gene": "UniProtKB:Q9ULZ0"
}